{
  "term_id": "GO:0016197",
  "gene_name": "Vacuolar protein sorting-associated protein 4B",
  "gene_symbol": "VPS4B",
  "term_label": "endosomal transport",
  "gene": "UniProtKB:O75351"
}